{
  "term_label": "MAP kinase kinase kinase activity",
  "gene_name": "Mitogen-activated protein kinase kinase kinase 7",
  "term_id": "GO:0004709",
  "gene": "UniProtKB:O43318",
  "gene_symbol": "MAP3K7"
}